{
  "gene": "UniProtKB:Q9Y2T1",
  "term_label": "plasma membrane",
  "gene_name": "Axin-2",
  "term_id": "GO:0005886",
  "gene_symbol": "AXIN2"
}